{
  "gene_symbol": "FAM110C",
  "gene": "UniProtKB:Q1W6H9",
  "term_id": "GO:0060491",
  "term_label": "regulation of cell projection assembly",
  "gene_name": "Protein FAM110C"
}